N-acetylornithine carbamoyltransferase activity [GO:0043857] (molecular function) Definition: Catalysis of the reaction: N(2)-acetyl-L-ornithine + carbamoyl phosphate = N(2)-acetyl-L-citrulline + H+ + phosphate. Also known as: N-acetylornithine transcarbamylase activity, acetylornithine transcarbamylase activity, AOTC, carbamoyl-phosphate:2-N-acetyl-L-ornithine carbamoyltransferase activity, carbamoyl-phosphate:N2-acetyl-L-ornithine carbamoyltransferase activity Relationships: is a type of carboxyl- or carbamoyltransferase activity [GO:0016743] Sources: EC:2.1.3.9, RHEA:18609